{
  "term_id": "GO:0030156",
  "gene_symbol": "RIMBP3C",
  "gene_name": "RIMS-binding protein 3C",
  "term_label": "benzodiazepine receptor binding",
  "gene": "UniProtKB:A6NJZ7"
}